{
  "term_id": "GO:0097194",
  "gene": "UniProtKB:Q96NN9",
  "gene_symbol": "AIFM3",
  "gene_name": "Apoptosis-inducing factor 3",
  "term_label": "execution phase of apoptosis"
}